{
  "gene": "UniProtKB:P0CJ86",
  "term_id": "GO:0006357",
  "term_label": "regulation of transcription by RNA polymerase II",
  "gene_name": "Double homeobox protein 4-like protein 3",
  "gene_symbol": "DUX4L3"
}